{
  "gene_symbol": "ADH1B",
  "gene": "UniProtKB:P00325",
  "term_label": "retinol metabolic process",
  "gene_name": "All-trans-retinol dehydrogenase [NAD(+)] ADH1B",
  "term_id": "GO:0042572"
}